polyterpenoid catabolic process [GO:0016113] (biological process) Relationships: is a type of terpenoid catabolic process [GO:0016115] Also known as: polyterpenoid breakdown, polyterpenoid catabolism, polyterpenoid degradation, polyterpene catabolic process, polyterpene catabolism Sources: GOC:go_curators Definition: The chemical reactions and pathways resulting in the breakdown of polyterpenoid compounds, terpenoids with more than eight isoprene units.